oocyte karyosome formation [GO:0030717] (biological process) References: PMID:11700288, PMID:18039935 Regulation: RO_0002211 by GO:0120313; negatively regulated by GO:0120314; positively regulated by positive regulation of oocyte karyosome formation [GO:0120315] Relationships: is a type of karyosome formation [GO:0061988]; is part of oogenesis [GO:0048477] Definition: The chromosome organization process in which meiotic chromosomes in the oocyte nucleus cluster together to form a compact spherical structure called the karyosome.